{
  "gene": "UniProtKB:Q18PE1",
  "term_id": "GO:0019901",
  "gene_symbol": "DOK7",
  "gene_name": "Protein Dok-7",
  "term_label": "protein kinase binding"
}